nose development [GO:0043584] (biological process) Sources: GOC:jl Definition: The process whose specific outcome is the progression of the nose over time, from its formation to the mature structure. The nose is the specialized structure of the face that serves as the organ of the sense of smell and as part of the respiratory system. Includes the nasi externus (external nose) and cavitas nasi (nasal cavity). Relationships: is a type of GO:0007423; is part of GO:0060541 Also known as: nasus development